{
  "term_label": "Unknown biological process",
  "gene_symbol": "FAM204A",
  "gene_name": "Protein FAM204A",
  "gene": "UniProtKB:Q9H8W3",
  "term_id": "UNKNOWN:0002"
}